glucuronoxylan metabolic process [GO:0010413] (biological process) Relationships: is a type of xylan metabolic process [GO:0045491] Sources: GOC:tair_curators Also known as: glucuronoxylan metabolism Subtypes: glucuronoxylan biosynthetic process [GO:0010417], glucuronoxylan catabolic process [GO:2000886] Definition: The chemical reactions and pathways involving xylan, a polymer containing a beta-(1->4)-linked D-xylose backbone decorated with glucuronic acid side units.